{
  "term_label": "mitochondrion",
  "gene_name": "HIG1 domain family member 1C",
  "term_id": "GO:0005739",
  "gene": "UniProtKB:A8MV81",
  "gene_symbol": "HIGD1C"
}